{
  "term_label": "membrane",
  "gene": "UniProtKB:Q8IZK6",
  "term_id": "GO:0016020",
  "gene_name": "Mucolipin-2",
  "gene_symbol": "MCOLN2"
}